{
  "term_label": "immune response",
  "term_id": "GO:0006955",
  "gene_symbol": "HLA-A",
  "gene": "UniProtKB:P04439",
  "gene_name": "HLA class I histocompatibility antigen, A alpha chain"
}